cellular response to glucagon stimulus [GO:0071377] (biological process) Definition: Any process that results in a change in state or activity of a cell (in terms of movement, secretion, enzyme production, gene expression, etc.) as a result of a glucagon stimulus. Sources: GOC:mah Relationships: is a type of response to glucagon [GO:0033762]; is_a cellular response to peptide hormone stimulus [GO:0071375]